negative regulation of abscisic acid-activated signaling pathway [GO:0009788] (biological process) Relationships: is a type of regulation of abscisic acid-activated signaling pathway [GO:0009787]; is a type of GO:0009968; is a type of negative regulation of cellular response to alcohol [GO:1905958]; negatively regulates abscisic acid-activated signaling pathway [GO:0009738] Also known as: down regulation of abscisic acid mediated signaling, down-regulation of abscisic acid mediated signaling, downregulation of abscisic acid mediated signaling, negative regulation of abscisic acid mediated signalling, inhibition of abscisic acid mediated signaling, negative regulation of abscisic acid mediated signaling pathway Sources: GOC:lr Definition: Any process that stops, prevents, or reduces the frequency, rate or extent of abscisic acid (ABA) signaling.